{
  "gene_name": "Protein Flattop",
  "gene": "UniProtKB:Q5VTH2",
  "term_label": "Unknown molecular function",
  "term_id": "UNKNOWN:0001",
  "gene_symbol": "CFAP126"
}